{
  "gene": "UniProtKB:P0CG40",
  "gene_name": "Transcription factor Sp9",
  "gene_symbol": "SP9",
  "term_id": "GO:0000981",
  "term_label": "DNA-binding transcription factor activity, RNA polymerase II-specific"
}